{
  "gene_name": "Matrix metalloproteinase-20",
  "gene": "UniProtKB:O60882",
  "term_id": "GO:0004222",
  "term_label": "metalloendopeptidase activity",
  "gene_symbol": "MMP20"
}